{
  "term_label": "RNA polymerase II cis-regulatory region sequence-specific DNA binding",
  "gene_symbol": "HOXB6",
  "term_id": "GO:0000978",
  "gene_name": "Homeobox protein Hox-B6",
  "gene": "UniProtKB:P17509"
}